{
  "term_id": "GO:0047734",
  "term_label": "CDP-glycerol diphosphatase activity",
  "gene": "UniProtKB:Q3LIE5",
  "gene_symbol": "ADPRM",
  "gene_name": "Manganese-dependent ADP-ribose_CDP-alcohol diphosphatase"
}